{
  "gene_name": "Insulin receptor substrate 2",
  "term_id": "GO:0005886",
  "term_label": "plasma membrane",
  "gene_symbol": "IRS2",
  "gene": "UniProtKB:Q9Y4H2"
}